{
  "gene": "UniProtKB:Q8HWS3",
  "term_label": "DNA-binding transcription factor activity, RNA polymerase II-specific",
  "gene_symbol": "RFX6",
  "gene_name": "DNA-binding protein RFX6",
  "term_id": "GO:0000981"
}